digestive hormone activity [GO:0046659] (MF) Definition: The action characteristic of a hormone that takes part in the digestion process. Also known as: secretin Sources: GOC:ai Relationships: is a type of hormone activity [GO:0005179]